N-methylphosphoethanolamine cytidylyltransferase activity [GO:0047353] (molecular function) Relationships: is a type of cytidylyltransferase activity [GO:0070567] Also known as: CTP:N-methylphosphoethanolamine cytidylyltransferase activity, CTP:N-methylethanolamine-phosphate cytidylyltransferase activity, CTP:P-MEA cytidylyltransferase activity, monomethylethanolamine phosphate cytidylyltransferase activity Sources: EC:2.7.7.57, RHEA:10576 Definition: Catalysis of the reaction: N-methylethanolamine phosphate + CTP = CDP-N-methylethanolamine + diphosphate.